parallel fiber to Purkinje cell synapse [GO:0098688] (cellular component) References: PMID:16623829, PMID:3209740 Relationships: is a type of GO:0060076 Definition: An excitatory synapse formed by the parallel fibers of granule cells synapsing onto the dendrites of Purkinje cells.